{
  "gene": "UniProtKB:P29692",
  "gene_symbol": "EEF1D",
  "term_id": "GO:0006414",
  "term_label": "translational elongation",
  "gene_name": "Elongation factor 1-delta"
}